{
  "gene_name": "Beta-2 adrenergic receptor",
  "gene": "UniProtKB:P07550",
  "gene_symbol": "ADRB2",
  "term_id": "GO:0004941",
  "term_label": "beta2-adrenergic receptor activity"
}